{
  "gene": "UniProtKB:P35250",
  "gene_name": "Replication factor C subunit 2",
  "term_id": "GO:0006281",
  "gene_symbol": "RFC2",
  "term_label": "DNA repair"
}